{
  "term_id": "GO:0005886",
  "gene": "UniProtKB:P25391",
  "gene_name": "Laminin subunit alpha-1",
  "term_label": "plasma membrane",
  "gene_symbol": "LAMA1"
}